{
  "term_label": "cytoskeleton",
  "gene_symbol": "KRT16",
  "gene": "UniProtKB:P08779",
  "gene_name": "Keratin, type I cytoskeletal 16",
  "term_id": "GO:0005856"
}